{
  "gene_name": "Elongator complex protein 4",
  "term_label": "cytoplasm",
  "gene_symbol": "ELP4",
  "gene": "UniProtKB:Q96EB1",
  "term_id": "GO:0005737"
}